3-methylquercitin 7-O-methyltransferase activity [GO:0030757] (molecular function) Definition: Catalysis of the reaction: 3',4',5,7-tetrahydroxy-3-methoxyflavone + S-adenosyl-L-methionine(1+) = 3',4',5-trihydroxy-3,7-dimethoxyflavone + S-adenosyl-L-homocysteine. Sources: EC:2.1.1.82, RHEA:16181 Also known as: 3-methylquercetin 7-O-methyltransferase activity, 7-OMT activity, S-adenosyl-L-methionine:3',4',5,7-tetrahydroxy-3-methoxyflavone 7-O-methyltransferase activity, S-adenosyl-L-methionine:5,7,3',4'-tetrahydroxy-3-methoxyflavone 7-O-methyltransferase activity, flavonol 7-O-methyltransferase activity, flavonol 7-methyltransferase activity Relationships: is a type of S-adenosylmethionine-dependent methyltransferase activity [GO:0008757]